posterior lateral line neuromast support cell differentiation [GO:0048927] (biological process) Definition: The process in which a relatively unspecialized cell acquires specialized features of a posterior lateral line neuromast support cell. Support cells are non-sensory cells of the neuromast that extend between the sensory hair cells from the basement membrane to the apical surface; they are surrounded by mantle cells. Sources: ISBN:0387968377 Relationships: is a type of neuromast support cell differentiation [GO:0048889]; is part of posterior lateral line neuromast development [GO:0048919]